{
  "gene_name": "OX-2 membrane glycoprotein",
  "term_id": "GO:0009986",
  "gene_symbol": "CD200",
  "gene": "UniProtKB:P41217",
  "term_label": "cell surface"
}